{
  "term_label": "Unknown molecular function",
  "gene_symbol": "TRB",
  "gene_name": "T cell receptor beta chain MC.7.G5",
  "term_id": "UNKNOWN:0001",
  "gene": "UniProtKB:P0DTU4"
}